{
  "term_label": "Unknown biological process",
  "term_id": "UNKNOWN:0002",
  "gene_symbol": "CMSS1",
  "gene_name": "Protein CMSS1",
  "gene": "UniProtKB:Q9BQ75"
}